inorganic triphosphate phosphatase activity [GO:0050355] (molecular function) Sources: EC:3.6.1.25, RHEA:14157 Definition: Catalysis of the reaction: H2O + inorganic triphosphate = diphosphate + phosphate. Also known as: triphosphatase activity, tripolyphosphatase activity, inorganic triphosphatase activity, triphosphate phosphohydrolase activity Relationships: is a type of pyrophosphatase activity [GO:0016462]